{
  "term_label": "Unknown molecular function",
  "term_id": "UNKNOWN:0001",
  "gene_symbol": "ULK4",
  "gene_name": "Serine_threonine-protein kinase ULK4",
  "gene": "UniProtKB:Q96C45"
}